{
  "term_id": "GO:0051015",
  "term_label": "actin filament binding",
  "gene_symbol": "WDR1",
  "gene": "UniProtKB:O75083",
  "gene_name": "WD repeat-containing protein 1"
}